{
  "gene_name": "Sodium channel protein type 10 subunit alpha",
  "gene_symbol": "SCN10A",
  "term_id": "GO:0005248",
  "gene": "UniProtKB:Q9Y5Y9",
  "term_label": "voltage-gated sodium channel activity"
}